{
  "term_label": "plasma membrane",
  "gene_symbol": "CD160",
  "gene": "UniProtKB:O95971",
  "term_id": "GO:0005886",
  "gene_name": "CD160 antigen"
}